{
  "gene_symbol": "PLXNB3",
  "gene": "UniProtKB:Q9ULL4",
  "gene_name": "Plexin-B3",
  "term_label": "negative regulation of cell adhesion",
  "term_id": "GO:0007162"
}